{
  "gene_symbol": "PRR20D",
  "term_id": "UNKNOWN:0001",
  "gene": "UniProtKB:P86480",
  "gene_name": "Proline-rich protein 20D",
  "term_label": "Unknown molecular function"
}